{
  "term_label": "mitochondrion",
  "gene_symbol": "COQ10A",
  "gene_name": "Coenzyme Q-binding protein COQ10 homolog A, mitochondrial",
  "term_id": "GO:0005739",
  "gene": "UniProtKB:Q96MF6"
}